{
  "gene": "UniProtKB:Q9NY27",
  "term_id": "GO:0005634",
  "gene_symbol": "PPP4R2",
  "term_label": "nucleus",
  "gene_name": "Serine_threonine-protein phosphatase 4 regulatory subunit 2"
}